{
  "gene": "UniProtKB:Q6UXS9",
  "gene_symbol": "CASP12",
  "term_id": "GO:0072558",
  "gene_name": "Inactive caspase-12",
  "term_label": "NLRP1 inflammasome complex"
}